{
  "gene_symbol": "SLC19A2",
  "gene_name": "Thiamine transporter 1",
  "term_id": "GO:0005886",
  "gene": "UniProtKB:O60779",
  "term_label": "plasma membrane"
}